{
  "term_id": "UNKNOWN:0002",
  "term_label": "Unknown biological process",
  "gene_symbol": "USP17L23",
  "gene": "UniProtKB:D6RBM5",
  "gene_name": "Putative ubiquitin carboxyl-terminal hydrolase 17-like protein 23"
}